{
  "term_label": "Unknown molecular function",
  "gene_name": "COMM domain-containing protein 9",
  "term_id": "UNKNOWN:0001",
  "gene": "UniProtKB:Q9P000",
  "gene_symbol": "COMMD9"
}